{
  "term_label": "Golgi apparatus",
  "gene_symbol": "GALNT7",
  "gene": "UniProtKB:Q86SF2",
  "gene_name": "N-acetylgalactosaminyltransferase 7",
  "term_id": "GO:0005794"
}